{
  "term_label": "nucleus",
  "term_id": "GO:0005634",
  "gene_symbol": "ZNF764",
  "gene_name": "Zinc finger protein 764",
  "gene": "UniProtKB:Q96H86"
}